{
  "term_label": "chloride transmembrane transporter activity",
  "gene": "UniProtKB:O95258",
  "term_id": "GO:0015108",
  "gene_name": "Brain mitochondrial carrier protein 1",
  "gene_symbol": "SLC25A14"
}